cytoplasmic polyadenylation-dependent RNA catabolic process [GO:0180018] (biological process) Relationships: is a type of polyadenylation-dependent RNA catabolic process [GO:0043633] References: PMID:20368444 Subtypes: cytoplasmic polyadenylation-dependent rRNA catabolic process [GO:0035760] Definition: The chemical reactions and pathways occurring in the cytoplasm and resulting in the breakdown of an RNA molecule, initiated by the enzymatic addition of a sequence of adenylyl residues (polyadenylation) at the 3' end the target rRNA truncated degradation intermediate.